{
  "gene_symbol": "DEFA5",
  "term_id": "GO:0050830",
  "term_label": "defense response to Gram-positive bacterium",
  "gene_name": "Defensin alpha 5",
  "gene": "UniProtKB:Q01523"
}